regulation of interleukin-37 production [GO:0150136] (biological process) References: PMID:30362558 Sources: GOC:aruk Definition: Any process that modulates the frequency, rate or extent of interleukin-37 production. Subtypes: negative regulation of interleukin-37 production [GO:0150138], positive regulation of interleukin-37 production [GO:0150139] Also known as: regulation of interleukin-37 biosynthetic process Relationships: is_a regulation of cytokine production [GO:0001817]; regulates interleukin-37 production [GO:0150137]